{
  "term_id": "GO:0005886",
  "gene_name": "Rap guanine nucleotide exchange factor 5",
  "gene": "UniProtKB:Q92565",
  "gene_symbol": "RAPGEF5",
  "term_label": "plasma membrane"
}